protein-succinyllysine desuccinylase activity [GO:0036055] (molecular function) Note: This reaction is the removal of a succinyl group (CO-CH2-CH2-CO) from a succinylated lysine residue of a protein or peptide. Relationships: is a type of NAD-dependent protein lysine deacylase activity [GO:0141218]; is part of peptidyl-lysine desuccinylation [GO:0036049] References: PMID:22076378 Sources: RHEA:47668 Also known as: succinyl lysine desuccinylase activity, succinyllysine desuccinylase activity, peptidyl-succinyllysine desuccinylase activity Definition: Catalysis of the reaction: N(6)-succinyl-L-lysyl-[protein] + NAD+ + H2O = 2''-O-succinyl-ADP-D-ribose + nicotinamide + L-lysyl-[protein].